{
  "term_label": "plasma membrane",
  "gene": "UniProtKB:Q8IWV2",
  "term_id": "GO:0005886",
  "gene_symbol": "CNTN4",
  "gene_name": "Contactin-4"
}